{
  "gene": "UniProtKB:O60676",
  "term_label": "cell surface",
  "term_id": "GO:0009986",
  "gene_symbol": "CST8",
  "gene_name": "Cystatin-8"
}